{
  "gene": "UniProtKB:Q9H7Z3",
  "gene_name": "Nuclear exosome regulator NRDE2",
  "term_id": "GO:0031048",
  "gene_symbol": "NRDE2",
  "term_label": "regulatory ncRNA-mediated heterochromatin formation"
}